{
  "term_label": "Unknown molecular function",
  "term_id": "UNKNOWN:0001",
  "gene": "UniProtKB:Q86UX2",
  "gene_symbol": "ITIH5",
  "gene_name": "Inter-alpha-trypsin inhibitor heavy chain H5"
}